{
  "gene_symbol": "ZNF818P",
  "gene_name": "Putative zinc finger protein 818",
  "term_label": "Unknown biological process",
  "term_id": "UNKNOWN:0002",
  "gene": "UniProtKB:Q6ZRF7"
}